{
  "term_id": "GO:0005634",
  "gene": "UniProtKB:P61086",
  "term_label": "nucleus",
  "gene_symbol": "UBE2K",
  "gene_name": "Ubiquitin-conjugating enzyme E2 K"
}